meiotic sister chromatid segregation [GO:0045144] (biological process) Also known as: meiosis II, chromosome segregation Sources: GOC:ai, ISBN:0815316194 Definition: The cell cycle process in which sister chromatids are organized and then physically separated and randomly apportioned to two sets during the second division of the meiotic cell cycle. Relationships: is a type of sister chromatid segregation [GO:0000819]; is a type of meiotic chromosome segregation [GO:0045132]; is a type of chromosome organization involved in meiotic cell cycle [GO:0070192]; is part of meiosis II [GO:0007135]